{
  "gene_symbol": "GRHL2",
  "gene": "UniProtKB:Q6ISB3",
  "term_id": "GO:0021915",
  "gene_name": "Grainyhead-like protein 2 homolog",
  "term_label": "neural tube development"
}